phosphatidylglycerol metabolic process [GO:0046471] (biological process) Definition: The chemical reactions and pathways involving phosphatidylglycerols, any of a class of phospholipids in which the phosphatidyl group is esterified to the hydroxyl group of glycerol. They are important constituents of cell membranes. Sources: ISBN:0198506732 Also known as: phosphatidylglycerol metabolism Relationships: is a type of glycerophospholipid metabolic process [GO:0006650] Subtypes: GO:0006655, cardiolipin metabolic process [GO:0032048], GO:0034478, phosphatidylglycerol acyl-chain remodeling [GO:0036148]